{
  "gene_name": "Protein SSUH2 homolog",
  "term_id": "UNKNOWN:0003",
  "gene_symbol": "SSUH2",
  "term_label": "Unknown cellular component",
  "gene": "UniProtKB:Q9Y2M2"
}